{
  "term_id": "GO:0005794",
  "gene": "UniProtKB:Q6ICL7",
  "term_label": "Golgi apparatus",
  "gene_name": "Solute carrier family 35 member E4",
  "gene_symbol": "SLC35E4"
}